{
  "gene_name": "TOG array regulator of axonemal microtubules protein 1",
  "gene": "UniProtKB:Q9Y4F4",
  "term_id": "GO:0005881",
  "term_label": "cytoplasmic microtubule",
  "gene_symbol": "TOGARAM1"
}